{
  "gene_symbol": "PDGFC",
  "gene_name": "Platelet-derived growth factor C",
  "term_label": "positive regulation of phosphatidylinositol 3-kinase/protein kinase B signal transduction",
  "term_id": "GO:0051897",
  "gene": "UniProtKB:Q9NRA1"
}